{
  "term_id": "GO:0005829",
  "gene": "UniProtKB:Q96KE9",
  "term_label": "cytosol",
  "gene_name": "BTB_POZ domain-containing protein 6",
  "gene_symbol": "BTBD6"
}